{
  "term_id": "GO:0034625",
  "gene_name": "Elongation of very long chain fatty acids protein 4",
  "gene_symbol": "ELOVL4",
  "term_label": "fatty acid elongation, monounsaturated fatty acid",
  "gene": "UniProtKB:Q9GZR5"
}